dimethylallyltranstransferase activity [GO:0004161] (molecular function) Sources: RHEA:22408 Definition: Catalysis of the reaction: dimethylallyl diphosphate + isopentenyl diphosphate = (2E)-geranyl diphosphate + diphosphate. Note: Note that this is the first step in the formation of farnesyl diphosphate. The second step is 'geranyltranstransferase activity ; GO:0004337'. Consider also annotating to the biological process term 'farnesyl diphosphate biosynthetic process ; GO:0045337'. Also known as: dimethylallyltransferase activity, geranyl diphosphate synthase activity, (2E,6E)-farnesyl diphosphate synthetase activity, DMAPP:IPP-dimethylallyltransferase activity, dimethylallyl-diphosphate:isopentenyl-diphosphate dimethylallyltranstransferase activity, diprenyltransferase activity, geranyl pyrophosphate synthase activity, geranyl pyrophosphate synthetase activity, geranyl-diphosphate synthase activity, trans-farnesyl pyrophosphate synthetase activity Relationships: is a type of prenyl diphosphate synthase activity [GO:0120531]